{
  "term_id": "GO:0003085",
  "gene": "UniProtKB:P42785",
  "term_label": "negative regulation of systemic arterial blood pressure",
  "gene_name": "Lysosomal Pro-X carboxypeptidase",
  "gene_symbol": "PRCP"
}